nuclear envelope [GO:0005635] (cellular component) Relationships: is a type of organelle envelope [GO:0031967]; is part of nucleus [GO:0005634]; is part of endomembrane system [GO:0012505] Definition: The double lipid bilayer that encloses the nucleus, separating its contents from the cytoplasm. It consists of an inner and outer nuclear membrane, with an intermembrane space (20-40 nm wide, also called the perinuclear space) between them. The envelope is supported by the nuclear lamina and contains nuclear pore complexes, which regulate molecular transport. References: PMID:16164970 Sources: ISBN:0198547684